TFIIA-class transcription factor complex binding [GO:0001092] (molecular function) Also known as: TFIIA-class transcription factor binding Definition: Binding to a general RNA polymerase II transcription factor belonging to the TFIIA complex, one of the complexes involved in formation of the preinitiation complex (PIC) by RNA polymerase II and defined as a basal or general transcription factor. References: PMID:16858867 Sources: GOC:krc Relationships: is a type of RNA polymerase II general transcription initiation factor binding [GO:0001091]; is a type of protein-containing complex binding [GO:0044877]